{
  "term_label": "peptidyl-prolyl cis-trans isomerase activity",
  "gene": "UniProtKB:A0A075B767",
  "gene_symbol": "PPIAL4H",
  "term_id": "GO:0003755",
  "gene_name": "Peptidyl-prolyl cis-trans isomerase A-like 4H"
}